{
  "gene": "UniProtKB:P51582",
  "gene_symbol": "P2RY4",
  "gene_name": "P2Y purinoceptor 4",
  "term_id": "GO:0045030",
  "term_label": "G protein-coupled UTP receptor activity"
}